{
  "term_id": "UNKNOWN:0001",
  "term_label": "Unknown molecular function",
  "gene_name": "Dapper homolog 2",
  "gene": "UniProtKB:Q5SW24",
  "gene_symbol": "DACT2"
}